{
  "gene_name": "G patch domain-containing protein 8",
  "term_label": "Unknown biological process",
  "gene_symbol": "GPATCH8",
  "term_id": "UNKNOWN:0002",
  "gene": "UniProtKB:Q9UKJ3"
}